{
  "term_id": "GO:0004222",
  "gene": "UniProtKB:Q9UNA0",
  "gene_symbol": "ADAMTS5",
  "gene_name": "A disintegrin and metalloproteinase with thrombospondin motifs 5",
  "term_label": "metalloendopeptidase activity"
}